{
  "gene": "UniProtKB:Q14137",
  "gene_symbol": "BOP1",
  "gene_name": "Ribosome biogenesis protein BOP1",
  "term_id": "GO:0030687",
  "term_label": "preribosome, large subunit precursor"
}